regulation of interleukin-17-mediated signaling pathway [GO:1903881] (biological process) Definition: Any process that modulates the frequency, rate or extent of interleukin-17-mediated signaling pathway. Subtypes: negative regulation of interleukin-17-mediated signaling pathway [GO:1903882], positive regulation of interleukin-17-mediated signaling pathway [GO:1903883] References: PMID:20054338 Sources: GOC:TermGenie, GOC:krc, GO_REF:0000058 Relationships: is a type of GO:0001959; regulates GO:0097400 Also known as: regulation of IL-17-mediated signaling pathway, regulation of IL-17-mediated signalling pathway, regulation of interleukin-17-mediated signalling pathway